{
  "term_id": "UNKNOWN:0002",
  "gene_name": "Surfactant-associated protein 3",
  "gene": "UniProtKB:P0C7M3",
  "gene_symbol": "SFTA3",
  "term_label": "Unknown biological process"
}